ventral disc lateral crest [GO:0097591] (cellular component) Relationships: is a type of cellular anatomical structure [GO:0110165]; is part of ventral disc [GO:0097597] Note: Due to the asymmetric nature of the Giardia trophozoite, this term is defined spatially as the trophozoite is viewed from the dorsal side, with the two nuclei dorsal to the ventral disc, and the ventral disc toward the anterior. Definition: Fibrillar repetitive structure surrounding the ventral disc edge in Giardia species (trophozoite stage). The composition of the lateral crest is not fully known yet. Sources: GOC:giardia Also known as: lateral crest, ventral disk lateral crest